olfactory behavior [GO:0042048] (BP) Definition: The behavior of an organism in response to an odor. Subtypes: olfactory learning [GO:0008355] Sources: GOC:jid, GOC:pr Relationships: is a type of chemosensory behavior [GO:0007635] Also known as: behavioral response to scent, behavioral response to smell, behavioural response to odour, behavioural response to scent, behavioural response to smell, olfactory behaviour